{
  "term_label": "Unknown molecular function",
  "gene_name": "Dolichyl-diphosphooligosaccharide--protein glycosyltransferase 48 kDa subunit",
  "term_id": "UNKNOWN:0001",
  "gene": "UniProtKB:P39656",
  "gene_symbol": "DDOST"
}